lymphoid lineage cell migration [GO:0097534] (BP) References: PMID:22342843 Sources: GOC:pr Relationships: is a type of cell migration [GO:0016477] Subtypes: lymphoid lineage cell migration into thymus [GO:0097535] Also known as: lymphoid lineage restricted progenitor cell migration Definition: The orderly movement of a lymphoid lineage cell from one site to another. A lymphoid lineage cell, also called a lymphoid lineage restricted progenitor cell, is a progenitor cell restricted to the lymphoid lineage.